{
  "term_id": "GO:0005829",
  "gene_symbol": "TIPRL",
  "gene": "UniProtKB:O75663",
  "term_label": "cytosol",
  "gene_name": "TIP41-like protein"
}